zinc ion sensor activity [GO:0106219] (molecular function) Definition: Binding to and responding, e.g. by conformational change, to changes in the cellular level of zinc. Relationships: is a type of metal ion sensor activity [GO:0140784]; BFO_0000051 zinc ion binding [GO:0008270] References: PMID:31239353 Sources: GOC:vw